{
  "gene_symbol": "NEDD4L",
  "term_label": "neuron projection development",
  "gene": "UniProtKB:Q96PU5",
  "gene_name": "E3 ubiquitin-protein ligase NEDD4-like",
  "term_id": "GO:0031175"
}